{
  "term_label": "cholesterol transport",
  "gene_symbol": "STARD3NL",
  "term_id": "GO:0030301",
  "gene_name": "STARD3 N-terminal-like protein",
  "gene": "UniProtKB:O95772"
}